{
  "term_id": "GO:0007200",
  "gene": "UniProtKB:O94806",
  "gene_name": "Serine_threonine-protein kinase D3",
  "gene_symbol": "PRKD3",
  "term_label": "phospholipase C-activating G protein-coupled receptor signaling pathway"
}